{
  "gene": "UniProtKB:Q6UXX9",
  "gene_symbol": "RSPO2",
  "term_id": "GO:0005615",
  "gene_name": "R-spondin-2",
  "term_label": "extracellular space"
}